{
  "term_id": "GO:0140912",
  "gene_name": "Beta-defensin 125",
  "term_label": "membrane destabilizing activity",
  "gene": "UniProtKB:Q8N687",
  "gene_symbol": "DEFB125"
}